positive regulation of intracellular transport [GO:0032388] (biological process) Subtypes: positive regulation of intracellular lipid transport [GO:0032379], positive regulation of nucleocytoplasmic transport [GO:0046824], positive regulation of anterograde axonal transport of mitochondrion [GO:0061881], GO:0090316, positive regulation of vesicle transport along microtubule [GO:1901610], positive regulation of calcium ion import into sarcoplasmic reticulum [GO:1902082], GO:1902840, positive regulation of ER to Golgi vesicle-mediated transport [GO:1902953], positive regulation of early endosome to recycling endosome transport [GO:1902955], positive regulation of vacuolar transport [GO:1903337], positive regulation of dense core granule transport [GO:1904811], positive regulation of retrograde transport, endosome to Golgi [GO:1905281], positive regulation of intraciliary anterograde transport [GO:1905798], positive regulation of intraciliary retrograde transport [GO:1905801], positive regulation of early endosome to late endosome transport [GO:2000643], positive regulation of retrograde axon cargo transport [GO:2001019], positive regulation of endocytic recycling [GO:2001137] Relationships: is a type of GO:0032386; is_a positive regulation of cellular process [GO:0048522]; is a type of positive regulation of transport [GO:0051050]; positively regulates GO:0046907 Also known as: up regulation of intracellular transport, up-regulation of intracellular transport, upregulation of intracellular transport, activation of intracellular transport, stimulation of intracellular transport Sources: GOC:mah Definition: Any process that activates or increases the frequency, rate or extent of the directed movement of substances within cells.